{
  "gene_name": "Protein PRRC2C",
  "term_label": "Unknown cellular component",
  "term_id": "UNKNOWN:0003",
  "gene_symbol": "PRRC2C",
  "gene": "UniProtKB:Q9Y520"
}